{
  "term_label": "negative regulation of transcription by RNA polymerase II",
  "gene": "UniProtKB:A0A0J9YX57",
  "term_id": "GO:0000122",
  "gene_symbol": "MAGEB6B",
  "gene_name": "Melanoma-associated antigen B6B"
}